{
  "term_id": "GO:0000381",
  "gene_name": "Cytotoxic granule associated RNA binding protein TIA1",
  "term_label": "regulation of alternative mRNA splicing, via spliceosome",
  "gene": "UniProtKB:P31483",
  "gene_symbol": "TIA1"
}